{
  "term_id": "GO:0005886",
  "gene_symbol": "OR13F1",
  "gene_name": "Olfactory receptor 13F1",
  "gene": "UniProtKB:Q8NGS4",
  "term_label": "plasma membrane"
}